{
  "gene_symbol": "PKP2",
  "term_label": "adherens junction",
  "gene": "UniProtKB:Q99959",
  "term_id": "GO:0005912",
  "gene_name": "Plakophilin-2"
}